rhamnogalacturonan acetylesterase activity [GO:0046575] (molecular function) References: PMID:10801485 Definition: Catalysis of the removal of acetylesters (as acetate) from galacturonic acid residues in the backbone of rhamnogalacturonan. Relationships: is a type of acetylesterase activity [GO:0008126]